{
  "term_label": "Unknown molecular function",
  "gene_name": "Angiopoietin-related protein 5",
  "gene_symbol": "ANGPTL5",
  "term_id": "UNKNOWN:0001",
  "gene": "UniProtKB:Q86XS5"
}